{
  "gene_symbol": "PLEKHA8",
  "gene": "UniProtKB:Q96JA3",
  "term_label": "cytosol",
  "gene_name": "Pleckstrin homology domain-containing family A member 8",
  "term_id": "GO:0005829"
}